{
  "gene_name": "Zinc finger protein 777",
  "gene_symbol": "ZNF777",
  "gene": "UniProtKB:Q9ULD5",
  "term_id": "GO:0005634",
  "term_label": "nucleus"
}